response to thyrotropin-releasing hormone [GO:1905225] (biological process) References: PMID:21382270 Sources: GOC:TermGenie, GOC:sl, GO_REF:0000071 Definition: Any process that results in a change in state or activity of a cell or an organism (in terms of movement, secretion, enzyme production, gene expression, etc.) as a result of a thyrotropin-releasing hormone (TRH) stimulus. TRH increases the secretion of thyroid-stimulating hormone by the anterior pituitary. Subtypes: cellular response to thyrotropin-releasing hormone [GO:1905229] Relationships: is a type of GO:0043434 Also known as: response to protirelin, response to TRH